{
  "gene": "UniProtKB:A4D256",
  "term_label": "cilium assembly",
  "gene_name": "Dual specificity protein phosphatase CDC14C",
  "term_id": "GO:0060271",
  "gene_symbol": "CDC14C"
}